{
  "gene": "UniProtKB:Q9BW91",
  "gene_symbol": "NUDT9",
  "term_label": "ADP-ribose diphosphatase activity",
  "gene_name": "ADP-ribose pyrophosphatase, mitochondrial",
  "term_id": "GO:0047631"
}